{
  "gene": "UniProtKB:Q9HB90",
  "term_label": "GTPase activity",
  "gene_name": "Ras-related GTP-binding protein C",
  "gene_symbol": "RRAGC",
  "term_id": "GO:0003924"
}